{
  "gene": "UniProtKB:Q92609",
  "gene_symbol": "TBC1D5",
  "term_id": "GO:0005096",
  "gene_name": "TBC1 domain family member 5",
  "term_label": "GTPase activator activity"
}